{
  "term_id": "GO:0008327",
  "gene": "UniProtKB:Q8WWY6",
  "term_label": "methyl-CpG binding",
  "gene_symbol": "MBD3L1",
  "gene_name": "Methyl-CpG-binding domain protein 3-like 1"
}